{
  "term_id": "GO:0048488",
  "gene": "UniProtKB:O15056",
  "term_label": "synaptic vesicle endocytosis",
  "gene_name": "Synaptojanin-2",
  "gene_symbol": "SYNJ2"
}